positive regulation of neural precursor cell proliferation [GO:2000179] (biological process) Definition: Any process that activates or increases the frequency, rate or extent of neural precursor cell proliferation. Sources: GOC:dph, GOC:yaf Relationships: is a type of positive regulation of cell population proliferation [GO:0008284]; is a type of regulation of neural precursor cell proliferation [GO:2000177]; positively regulates neural precursor cell proliferation [GO:0061351] Subtypes: GO:0002052, positive regulation of cerebellar granule cell precursor proliferation [GO:0021940], positive regulation of oligodendrocyte progenitor proliferation [GO:0070447], positive regulation of cell proliferation in dorsal spinal cord [GO:1902833], positive regulation of cell proliferation in midbrain [GO:1904935]